{
  "gene_name": "Unconventional myosin-Ig",
  "term_label": "actin filament binding",
  "gene_symbol": "MYO1G",
  "gene": "UniProtKB:B0I1T2",
  "term_id": "GO:0051015"
}